{
  "term_id": "GO:0036064",
  "gene_symbol": "DYNC2LI1",
  "gene_name": "Cytoplasmic dynein 2 light intermediate chain 1",
  "term_label": "ciliary basal body",
  "gene": "UniProtKB:Q8TCX1"
}